{
  "gene": "UniProtKB:Q96MH7",
  "term_label": "Unknown biological process",
  "gene_symbol": "C5orf34",
  "term_id": "UNKNOWN:0002",
  "gene_name": "Uncharacterized protein C5orf34"
}